larynx development [GO:0120224] (biological process) Relationships: is a type of animal organ development [GO:0048513]; is part of GO:0060541 Definition: The biological process whose specific outcome is the progression of a larynx from an initial condition to its mature state. This process begins with the formation of the larynx and ends with the mature structure. A larynx is a continuation of the pharynx that is involved in breathing, sound production, and protecting the trachea against food aspiration. References: PMID:28177282 Sources: GOC:krc